positive regulation of metabolic process [GO:0009893] (biological process) Also known as: positive regulation of metabolism, up regulation of metabolic process, up-regulation of metabolic process, upregulation of metabolic process, activation of metabolic process, positive regulation of multicellular organismal metabolic process, positive regulation of organismal metabolism, stimulation of metabolic process, stimulation of organismal metabolic process, up-regulation of organismal metabolic process Definition: Any process that activates or increases the frequency, rate or extent of the chemical reactions and pathways within a cell or an organism. Relationships: is a type of regulation of metabolic process [GO:0019222]; is a type of positive regulation of cellular process [GO:0048522]; positively regulates metabolic process [GO:0008152] Sources: GOC:go_curators Subtypes: GO:0009891, positive regulation of catabolic process [GO:0009896], positive regulation of phosphorus metabolic process [GO:0010562], positive regulation of macromolecule metabolic process [GO:0010604], positive regulation of collagen metabolic process [GO:0010714], GO:0031539, positive regulation of hormone metabolic process [GO:0032352], GO:0033240, positive regulation of amide metabolic process [GO:0034250], positive regulation of melanization defense response [GO:0035008], positive regulation of amino acid metabolic process [GO:0045764], positive regulation of lipid metabolic process [GO:0045834], GO:0045913, positive regulation of respiratory burst [GO:0060267], GO:0062013, GO:0106121, positive regulation of cold-induced thermogenesis [GO:0120162], positive regulation of sulfate assimilation [GO:1900059], positive regulation of cellular respiration [GO:1901857], positive regulation of nitrogen cycle metabolic process [GO:1903316], GO:1903705, GO:1905087, positive regulation of photosynthesis [GO:1905157], GO:1905448, positive regulation of reactive oxygen species metabolic process [GO:2000379]